DnaA-DnaB-DnaC complex [GO:1990157] (cellular component) References: PMID:20129058 Sources: GOC:bhm Definition: A protein-DNA complex consisting of the helicase loading complex DnaB-DnaC bound to the DNA-bound DNA replication initiation protein DnaA. Essential for DNA replication initiation. Relationships: is a type of pre-primosome complex [GO:1990099]; has part DnaB-DnaC complex [GO:1990100]